{
  "term_label": "histone demethylase activity",
  "gene": "UniProtKB:Q8NHM5",
  "gene_name": "Lysine-specific demethylase 2B",
  "gene_symbol": "KDM2B",
  "term_id": "GO:0032452"
}